4,8,12-trimethyltrideca-1,3,7,11-tetraene synthase activity [GO:0097007] (molecular function) Definition: Catalysis of the reaction: (EE)-geranyllinalool + NADPH + O2 = 4,8,12-trimethyl-1,3,7,11-tridecatetraene + NADP+ + 2 H2O. It is unknown whether this reaction proceeds by the direct release of the 4-carbon compound but-1-en-3-one, or whether the substrate is first degraded to C18-farnesylacetone and then cleaved to produce 4,8,12-trimethyl-1,3,7,11-tridecatetraene (TMTT) and acetone. Also known as: 4,8,12-trimethyl-1,3,7,11-tridecatetraene synthase activity, TMTT synthase activity References: PMID:21088219 Sources: GOC:kad, MetaCyc:RXN-8620 Relationships: is a type of GO:0016709